primary lung bud formation [GO:0060431] (biological process) Relationships: is a type of morphogenesis of embryonic epithelium [GO:0016331]; is a type of GO:0048645; is a type of epithelial tube branching involved in lung morphogenesis [GO:0060441]; is a type of GO:0060572 Also known as: lung formation Sources: GOC:dph, GOC:mtg_lung Definition: The morphogenetic process in which the foregut region specified to become the lung forms the initial left and right buds.